{
  "term_id": "GO:0006357",
  "term_label": "regulation of transcription by RNA polymerase II",
  "gene_name": "GA-binding protein alpha chain",
  "gene_symbol": "GABPA",
  "gene": "UniProtKB:Q06546"
}